{
  "gene_name": "Testis-expressed basic protein 1",
  "gene_symbol": "TSBP1",
  "term_id": "UNKNOWN:0002",
  "gene": "UniProtKB:Q5SRN2",
  "term_label": "Unknown biological process"
}